{
  "term_id": "GO:0042867",
  "term_label": "pyruvate catabolic process",
  "gene": "UniProtKB:P07864",
  "gene_symbol": "LDHC",
  "gene_name": "L-lactate dehydrogenase C chain"
}